{
  "gene": "UniProtKB:Q96RR4",
  "term_id": "GO:0004674",
  "gene_name": "Calcium_calmodulin-dependent protein kinase kinase 2",
  "term_label": "protein serine/threonine kinase activity",
  "gene_symbol": "CAMKK2"
}